{
  "term_id": "GO:0043495",
  "gene": "UniProtKB:Q676U5",
  "gene_name": "Autophagy-related protein 16-1",
  "term_label": "protein-membrane adaptor activity",
  "gene_symbol": "ATG16L1"
}